{
  "gene_name": "Cell cycle exit and neuronal differentiation protein 1",
  "term_id": "GO:0021933",
  "gene": "UniProtKB:Q8N111",
  "gene_symbol": "CEND1",
  "term_label": "radial glia guided migration of cerebellar granule cell"
}